N-(long-chain-acyl)ethanolamine deacylase activity [GO:0047412] (molecular function) Definition: Catalysis of the reaction: H2O + N-(long-chain-acyl)ethanolamine = ethanolamine + a fatty acid. Relationships: is a type of hydrolase activity, acting on carbon-nitrogen (but not peptide) bonds, in linear amides [GO:0016811] Also known as: N-(long-chain-acyl)ethanolamine amidohydrolase activity, N-acylethanolamine amidohydrolase activity, acylethanolamine amidase activity Sources: EC:3.5.1.60, MetaCyc:3.5.1.60-RXN